positive regulation of nematode pharynx morphogenesis [GO:0110043] (biological process) Definition: Any process that activates or increases the frequency, rate or extent of nematode pharynx morphogenesis. References: PMID:20805556 Sources: GOC:rz Relationships: is a type of regulation of nematode pharynx morphogenesis [GO:0110041]; is a type of positive regulation of animal organ morphogenesis [GO:0110110]; positively regulates GO:0110040